aminolevulinate transaminase activity [GO:0047665] (molecular function) Definition: Catalysis of the reaction: 5-aminolevulinate + pyruvate = 4,5-dioxopentanoate + L-alanine. Also known as: aminolevulinate aminotransferase activity, 4,5-dioxovalerate aminotransferase activity, 4,5-dioxovaleric acid aminotransferase activity, 4,5-dioxovaleric acid transaminase activity, 4,5-dioxovaleric transaminase activity, 5-aminolevulinate:pyruvate aminotransferase activity, 5-aminolevulinic acid transaminase activity, DOVA transaminase activity, L-alanine-4,5-dioxovalerate aminotransferase activity, L-alanine:4,5-dioxovaleric acid transaminase activity, L-alanine:dioxovalerate transaminase activity, alanine-dioxovalerate aminotransferase activity, alanine-gamma,delta-dioxovalerate aminotransferase activity, alanine:4,5-dioxovalerate aminotransferase activity, aminolevulinic acid transaminase activity, dioxovalerate transaminase activity, gamma,delta-dioxovalerate aminotransferase activity, gamma,delta-dioxovaleric acid transaminase activity Sources: EC:2.6.1.43, RHEA:12480 Relationships: is a type of transaminase activity [GO:0008483]